{
  "gene_symbol": "ZNF418",
  "term_id": "GO:0000981",
  "gene_name": "Zinc finger protein 418",
  "term_label": "DNA-binding transcription factor activity, RNA polymerase II-specific",
  "gene": "UniProtKB:Q8TF45"
}